{
  "term_label": "spermatid development",
  "gene_symbol": "RIMBP3B",
  "gene_name": "RIMS-binding protein 3B",
  "term_id": "GO:0007286",
  "gene": "UniProtKB:A6NNM3"
}